{
  "gene_symbol": "TIGD5",
  "gene_name": "Tigger transposable element-derived protein 5",
  "term_id": "GO:0005634",
  "gene": "UniProtKB:Q53EQ6",
  "term_label": "nucleus"
}